positive regulation of dopamine biosynthetic process [GO:1903181] (biological process) References: PMID:19703902 Sources: GOC:PARL, GOC:TermGenie, GOC:bf, GO_REF:0000058 Relationships: is a type of positive regulation of biosynthetic process [GO:0009891]; is a type of GO:0045964; is a type of regulation of dopamine biosynthetic process [GO:1903179]; positively regulates dopamine biosynthetic process [GO:0042416] Also known as: positive regulation of dopamine anabolism, positive regulation of dopamine biosynthesis, positive regulation of dopamine formation, positive regulation of dopamine synthesis, up regulation of dopamine anabolism, up regulation of dopamine biosynthesis, up regulation of dopamine biosynthetic process, up regulation of dopamine formation, up regulation of dopamine synthesis, up-regulation of dopamine anabolism, up-regulation of dopamine biosynthesis, up-regulation of dopamine biosynthetic process, up-regulation of dopamine formation, up-regulation of dopamine synthesis, upregulation of dopamine anabolism, upregulation of dopamine biosynthesis, upregulation of dopamine biosynthetic process, upregulation of dopamine formation, upregulation of dopamine synthesis, activation of dopamine anabolism, activation of dopamine biosynthesis, activation of dopamine biosynthetic process, activation of dopamine formation, activation of dopamine synthesis Definition: Any process that activates or increases the frequency, rate or extent of dopamine biosynthetic process.